myeloid leukocyte activation [GO:0002274] (biological process) Definition: A change in the morphology or behavior of a myeloid leukocyte resulting from exposure to an activating factor such as a cellular or soluble ligand. Subtypes: myeloid dendritic cell activation [GO:0001773], GO:0002275, granulocyte activation [GO:0036230], GO:0042116, monocyte activation [GO:0042117], mast cell activation [GO:0045576] Also known as: myeloid leucocyte activation Relationships: is a type of leukocyte activation [GO:0045321] Sources: GOC:add, ISBN:0781735149